{
  "term_id": "GO:0060170",
  "term_label": "ciliary membrane",
  "gene_name": "Limbin",
  "gene_symbol": "EVC2",
  "gene": "UniProtKB:Q86UK5"
}